{
  "term_label": "guanyl-nucleotide exchange factor activity",
  "gene_name": "Rho guanine nucleotide exchange factor 19",
  "term_id": "GO:0005085",
  "gene": "UniProtKB:Q8IW93",
  "gene_symbol": "ARHGEF19"
}